{
  "term_id": "GO:1990837",
  "gene": "UniProtKB:Q9BZM3",
  "gene_symbol": "GSX2",
  "term_label": "sequence-specific double-stranded DNA binding",
  "gene_name": "GS homeobox 2"
}